{
  "gene": "UniProtKB:P0DPK3",
  "gene_name": "Notch homolog 2 N-terminal-like protein B",
  "gene_symbol": "NOTCH2NLB",
  "term_label": "Notch binding",
  "term_id": "GO:0005112"
}